{
  "gene_name": "Ubiquitin-associated protein 2",
  "term_id": "GO:0005634",
  "term_label": "nucleus",
  "gene": "UniProtKB:Q5T6F2",
  "gene_symbol": "UBAP2"
}